{
  "term_label": "regulation of transcription by RNA polymerase II",
  "gene": "UniProtKB:Q7Z398",
  "gene_name": "Zinc finger protein 550",
  "term_id": "GO:0006357",
  "gene_symbol": "ZNF550"
}